secondary metabolite catabolic process [GO:0090487] (biological process) Sources: GOC:tb Also known as: secondary metabolite breakdown, secondary metabolite catabolism, secondary metabolite degradation Subtypes: polyketide catabolic process [GO:0030640], asperthecin catabolic process [GO:0036183], orcinol catabolic process [GO:0042209], penicillin catabolic process [GO:0042317], siderophore catabolic process [GO:0046215], GO:1900540, GO:1900550, emericellamide catabolic process [GO:1900556], GO:1900562, diorcinol catabolic process [GO:1900571], emodin catabolic process [GO:1900574], gerfelin catabolic process [GO:1900577], GO:1900580, GO:1900583, arugosin catabolic process [GO:1900586], GO:1900589, violaceol II catabolic process [GO:1900592], (+)-kotanin catabolic process [GO:1900595], GO:1900598, endocrocin catabolic process [GO:1900601], tensidol A catabolic process [GO:1900604], tensidol B catabolic process [GO:1900607], GO:1900765, GO:1900792, cordyol C catabolic process [GO:1900798], cspyrone B1 catabolic process [GO:1900801], helvolic acid catabolic process [GO:1900811], monodictyphenone catabolic process [GO:1900814], ochratoxin A catabolic process [GO:1900817], orlandin catabolic process [GO:1900820] Relationships: is_a catabolic process [GO:0009056]; is a type of secondary metabolic process [GO:0019748] Definition: The chemical reactions and pathways resulting in the breakdown of secondary metabolites, the compounds that are not necessarily required for growth and maintenance of cells, and are often unique to a taxon.